interleukin-17E receptor binding [GO:0030380] (molecular function) Also known as: IL-17E, interleukin-17E receptor ligand Relationships: is_a cytokine receptor binding [GO:0005126] Definition: Binding to an interleukin-17E receptor. Sources: GOC:ai